triphosphoribosyl-dephospho-CoA synthase activity [GO:0046917] (molecular function) Sources: EC:2.4.2.52 Also known as: ATP:3-dephospho-CoA 5''-triphosphoribosyltransferase activity, ATP:dephospho-CoA 5-triphosphoribosyl transferase activity, 2'-(5''-triphosphoribosyl)-3-dephospho-CoA synthase activity, CitG activity Definition: Catalysis of the reaction: ATP + 3-dephospho-CoA = 2'-(5''-triphosphoribosyl)-3'-dephospho-CoA + adenine. Relationships: is a type of GO:0016780